{
  "term_label": "cytosol",
  "gene_name": "G-protein coupled receptor-associated sorting protein 2",
  "gene": "UniProtKB:Q96D09",
  "term_id": "GO:0005829",
  "gene_symbol": "GPRASP2"
}